{
  "term_id": "GO:0005634",
  "gene_name": "Zinc finger protein 445",
  "gene_symbol": "ZNF445",
  "gene": "UniProtKB:P59923",
  "term_label": "nucleus"
}